{
  "gene_symbol": "SCN3A",
  "term_id": "GO:0086002",
  "term_label": "cardiac muscle cell action potential involved in contraction",
  "gene_name": "Sodium channel protein type 3 subunit alpha",
  "gene": "UniProtKB:Q9NY46"
}